male germ cell nucleus [GO:0001673] (cellular component) Also known as: male germ-cell nucleus Definition: The nucleus of a male germ cell, a reproductive cell in males. Relationships: is a type of GO:0043073 Sources: CL:0000015, GOC:hjd, GOC:mtg_sensu